{
  "term_label": "P-body",
  "gene": "UniProtKB:Q86TB9",
  "gene_name": "Protein PAT1 homolog 1",
  "gene_symbol": "PATL1",
  "term_id": "GO:0000932"
}